{
  "term_id": "GO:0016020",
  "gene": "UniProtKB:Q8NGC2",
  "gene_name": "Olfactory receptor 4E2",
  "term_label": "membrane",
  "gene_symbol": "OR4E2"
}